symbiont-mediated suppression of host chemokine signal transduction pathway [GO:0141135] (biological process) References: PMID:16581912 Relationships: is a type of symbiont-mediated suppression of host G protein-coupled receptor signal transduction [GO:0075120] Definition: A process in which a symbiont interferes with, inhibits or disrupts a chemokine signaling pathway, a G protein-coupled receptor signal transduction pathway activated by a chemokine. The host is defined as the larger of the organisms involved in a symbiotic interaction.